GDP-mannose transmembrane transport [GO:1990570] (biological process) Also known as: GDP-mannose transport Definition: The process in which GDP-mannose is transported across a membrane. Relationships: is a type of GO:0090480 References: PMID:9395539